{
  "gene_name": "Zinc finger protein 846",
  "gene_symbol": "ZNF846",
  "term_label": "regulation of transcription by RNA polymerase II",
  "term_id": "GO:0006357",
  "gene": "UniProtKB:Q147U1"
}